{
  "gene_symbol": "SEPTIN2",
  "term_label": "cytoskeleton-dependent cytokinesis",
  "term_id": "GO:0061640",
  "gene": "UniProtKB:Q15019",
  "gene_name": "Septin-2"
}